{
  "gene_symbol": "WIPF2",
  "term_label": "Unknown molecular function",
  "gene": "UniProtKB:Q8TF74",
  "gene_name": "WAS_WASL-interacting protein family member 2",
  "term_id": "UNKNOWN:0001"
}